{
  "term_label": "telomere localization",
  "term_id": "GO:0034397",
  "gene": "UniProtKB:Q8N6L0",
  "gene_symbol": "KASH5",
  "gene_name": "Protein KASH5"
}